{
  "gene": "UniProtKB:A0A0J9YX35",
  "gene_symbol": "IGHV3-64D",
  "term_label": "antigen binding",
  "gene_name": "Immunoglobulin heavy variable 3-64D",
  "term_id": "GO:0003823"
}